{
  "gene": "UniProtKB:Q9NRW1",
  "gene_name": "Ras-related protein Rab-6B",
  "term_label": "endomembrane system",
  "term_id": "GO:0012505",
  "gene_symbol": "RAB6B"
}